{
  "gene_name": "Dual specificity tyrosine-phosphorylation-regulated kinase 1A",
  "gene_symbol": "DYRK1A",
  "term_id": "GO:0045893",
  "term_label": "positive regulation of DNA-templated transcription",
  "gene": "UniProtKB:Q13627"
}